symbiont-mediated evasion of mRNA degradation by host via mRNA cap methylation [GO:0039699] (biological process) Definition: An innate immune response evasion mechanism in which a symbiont methylates the 2'-O-ribose of the first or second transcribed nucleotide of its mRNAs. Methylation allows evasion of the host innate immune response, which degrades cap0 (non-methylated) mRNAs. This mechanism of immune evasion is used by viruses. References: PMID:35215972 Also known as: IFIT mRNA restriction evasion by virus, evasion of mRNA degradation by host via mRNA cap methylation, viral mRNA cap methylation Relationships: is a type of GO:0141177